{
  "gene_symbol": "PRSS23",
  "term_id": "UNKNOWN:0001",
  "gene": "UniProtKB:O95084",
  "gene_name": "Serine protease 23",
  "term_label": "Unknown molecular function"
}